{
  "gene": "UniProtKB:Q9BWT3",
  "term_label": "Unknown biological process",
  "gene_name": "Poly(A) polymerase gamma",
  "term_id": "UNKNOWN:0002",
  "gene_symbol": "PAPOLG"
}